{
  "gene": "UniProtKB:P35222",
  "gene_symbol": "CTNNB1",
  "term_id": "GO:0016342",
  "term_label": "catenin complex",
  "gene_name": "Catenin beta-1"
}